{
  "gene_symbol": "PENK",
  "gene": "UniProtKB:P01210",
  "term_label": "neuropeptide signaling pathway",
  "gene_name": "Proenkephalin-A",
  "term_id": "GO:0007218"
}